N-carbamoyl-L-amino-acid hydrolase activity [GO:0050538] (molecular function) Definition: Catalysis of the reaction: N-carbamoyl-L-2-amino acid + H2O = L-2-amino acid + NH3 + CO2. The N-carbamoyl-L-2-amino acid is a 2-ureido carboxylate. Sources: EC:3.5.1.87, MetaCyc:3.5.1.87-RXN Also known as: L-carbamoylase activity, N-carbamoyl-L-amino acid amidohydrolase activity Relationships: is a type of hydrolase activity, acting on carbon-nitrogen (but not peptide) bonds, in linear amides [GO:0016811]